{
  "gene_name": "Sushi repeat-containing protein SRPX",
  "gene": "UniProtKB:P78539",
  "term_id": "UNKNOWN:0001",
  "gene_symbol": "SRPX",
  "term_label": "Unknown molecular function"
}